{
  "term_label": "skeletal muscle thin filament assembly",
  "term_id": "GO:0030240",
  "gene": "UniProtKB:O15273",
  "gene_name": "Telethonin",
  "gene_symbol": "TCAP"
}